{
  "term_id": "GO:0061630",
  "term_label": "ubiquitin protein ligase activity",
  "gene_symbol": "RCHY1",
  "gene": "UniProtKB:Q96PM5",
  "gene_name": "RING finger and CHY zinc finger domain-containing protein 1"
}